{
  "term_id": "UNKNOWN:0003",
  "gene_symbol": "SH3TC2",
  "gene": "UniProtKB:Q8TF17",
  "gene_name": "SH3 domain and tetratricopeptide repeat-containing protein 2",
  "term_label": "Unknown cellular component"
}